{
  "gene": "UniProtKB:Q9Y278",
  "gene_name": "Heparan sulfate glucosamine 3-O-sulfotransferase 2",
  "term_id": "GO:0008467",
  "gene_symbol": "HS3ST2",
  "term_label": "[heparan sulfate]-glucosamine 3-sulfotransferase activity"
}